{
  "gene_name": "Tumor necrosis factor receptor superfamily member 3",
  "gene": "UniProtKB:P36941",
  "gene_symbol": "LTBR",
  "term_id": "GO:0043123",
  "term_label": "positive regulation of canonical NF-kappaB signal transduction"
}